{
  "gene": "UniProtKB:Q7Z7A1",
  "gene_symbol": "CNTRL",
  "gene_name": "Centriolin",
  "term_id": "UNKNOWN:0002",
  "term_label": "Unknown biological process"
}